{
  "gene": "UniProtKB:Q9H0T7",
  "gene_symbol": "RAB17",
  "term_label": "endomembrane system",
  "term_id": "GO:0012505",
  "gene_name": "Ras-related protein Rab-17"
}